{
  "term_id": "GO:0030091",
  "gene": "UniProtKB:Q9NZV6",
  "gene_symbol": "MSRB1",
  "term_label": "protein repair",
  "gene_name": "Methionine-R-sulfoxide reductase B1"
}